{
  "term_id": "GO:0000127",
  "gene_symbol": "GTF3C4",
  "gene": "UniProtKB:Q9UKN8",
  "gene_name": "General transcription factor 3C polypeptide 4",
  "term_label": "transcription factor TFIIIC complex"
}